{
  "gene": "UniProtKB:O75509",
  "gene_name": "Tumor necrosis factor receptor superfamily member 21",
  "term_id": "GO:0031642",
  "term_label": "negative regulation of myelination",
  "gene_symbol": "TNFRSF21"
}